{
  "gene": "UniProtKB:O00178",
  "term_id": "GO:0003746",
  "gene_name": "GTP-binding protein 1",
  "term_label": "translation elongation factor activity",
  "gene_symbol": "GTPBP1"
}